{
  "gene": "UniProtKB:Q7Z553",
  "gene_name": "MAM domain-containing glycosylphosphatidylinositol anchor protein 2",
  "gene_symbol": "MDGA2",
  "term_label": "nervous system development",
  "term_id": "GO:0007399"
}